{
  "gene": "UniProtKB:Q58F21",
  "gene_symbol": "BRDT",
  "term_id": "GO:0003682",
  "gene_name": "Bromodomain testis-specific protein",
  "term_label": "chromatin binding"
}